{
  "gene_name": "Homeobox protein ARX",
  "term_id": "GO:0000981",
  "gene": "UniProtKB:Q96QS3",
  "gene_symbol": "ARX",
  "term_label": "DNA-binding transcription factor activity, RNA polymerase II-specific"
}